Par3-APC-KIF3A complex [GO:0034748] (cellular component) References: PMID:15556865 Relationships: is a type of protein-containing complex [GO:0032991]; is part of cytoplasm [GO:0005737] Note: Note that the gene/protein name 'APC' should not be confused with the abbreviation for 'anaphase promoting complex'. Definition: A protein complex that contains Par3, the tumor suppressor protein adenomatous polyposis coli (APC), and the kinesin-related protein KIF3A; involved in establishing neuronal cell polarity.